{
  "term_label": "nucleus",
  "gene": "UniProtKB:Q9UBP5",
  "gene_name": "Hairy_enhancer-of-split related with YRPW motif protein 2",
  "term_id": "GO:0005634",
  "gene_symbol": "HEY2"
}